protein localization to cell junction [GO:1902414] (biological process) Definition: A process in which a protein is transported to, or maintained in, a location within a cell junction. References: PMID:18332111 Sources: GOC:TermGenie Also known as: protein localisation in cell junction, protein localisation to cell junction, protein localization in cell junction Relationships: is a type of intracellular protein localization [GO:0008104] Subtypes: protein localization to synapse [GO:0035418], protein localization to cell-cell junction [GO:0150105]